{
  "gene_symbol": "MAGEA12",
  "term_id": "GO:0000122",
  "gene_name": "Melanoma-associated antigen 12",
  "gene": "UniProtKB:P43365",
  "term_label": "negative regulation of transcription by RNA polymerase II"
}